{
  "gene": "UniProtKB:Q8N3Y3",
  "term_label": "protein O-linked glycosylation via mannose",
  "gene_name": "Xylosyl- and glucuronyltransferase LARGE2",
  "term_id": "GO:0035269",
  "gene_symbol": "LARGE2"
}